{
  "term_id": "GO:0090575",
  "gene_symbol": "NR1H4",
  "gene": "UniProtKB:Q96RI1",
  "term_label": "RNA polymerase II transcription regulator complex",
  "gene_name": "Bile acid receptor"
}